{
  "term_label": "positive regulation of DNA-templated transcription, elongation",
  "term_id": "GO:0032786",
  "gene_name": "Cyclin-T1",
  "gene": "UniProtKB:O60563",
  "gene_symbol": "CCNT1"
}